{
  "term_id": "GO:0036064",
  "gene_name": "Kinocilin",
  "gene": "UniProtKB:A6PVL3",
  "term_label": "ciliary basal body",
  "gene_symbol": "KNCN"
}